{
  "term_id": "GO:0050911",
  "gene_symbol": "OR2I1",
  "gene": "UniProtKB:Q8NGU4",
  "term_label": "detection of chemical stimulus involved in sensory perception of smell",
  "gene_name": "Putative olfactory receptor 2I1"
}